{
  "gene_symbol": "CARMIL2",
  "term_id": "UNKNOWN:0001",
  "term_label": "Unknown molecular function",
  "gene": "UniProtKB:Q6F5E8",
  "gene_name": "Capping protein, Arp2_3 and myosin-I linker protein 2"
}